{
  "term_id": "GO:1905668",
  "gene": "UniProtKB:Q6PCB6",
  "gene_name": "Alpha_beta hydrolase domain-containing protein 17C",
  "term_label": "positive regulation of protein localization to endosome",
  "gene_symbol": "ABHD17C"
}